{
  "gene_name": "Polyamine-transporting ATPase 13A2",
  "gene": "UniProtKB:Q9NQ11",
  "term_label": "polyamine transmembrane transport",
  "gene_symbol": "ATP13A2",
  "term_id": "GO:1902047"
}